interstitial cell of Cajal differentiation [GO:0061453] (biological process) Definition: The process in which a relatively unspecialized cell acquires specialized features of an interstitial cell of Cajal. An interstitial cell of Cajal is an intestinal neuroepithelial cell that serves as a pacemaker to trigger gut contraction. Sources: GOC:dph Also known as: ICC differentiation Relationships: is a type of neuroepithelial cell differentiation [GO:0060563]; is a type of intestinal epithelial cell differentiation [GO:0060575]